homogentisate farnesyltransferase activity [GO:0010355] (MF) Definition: Catalysis of the reaction: homogentisic acid + farnesyl diphosphate = 2-methyl-6-farnesylplastoquinol. Relationships: is a type of GO:0010354 References: PMID:16989822